Ino80 complex [GO:0031011] (cellular component) References: PMID:19355820 Sources: GOC:jh, GOC:rb Definition: A multisubunit protein complex that contains the Ino80p ATPase; exhibits chromatin remodeling activity. Also known as: INO80 chromatin remodeling complex Relationships: is a type of INO80-type complex [GO:0097346]; is part of nuclear chromosome [GO:0000228]